{
  "gene_name": "Sorting nexin-5",
  "gene_symbol": "SNX5",
  "term_id": "GO:0035091",
  "gene": "UniProtKB:Q9Y5X3",
  "term_label": "phosphatidylinositol binding"
}